cyanidin 3-O-glucoside 7-O-glucosyltransferase (acyl-glucose) activity [GO:0102457] (molecular function) Relationships: is a type of GO:0016758 Also known as: cyanidin 3-O-glucoside 7-O-glucosyltransferase (vanilloyl-glucose dependent) activity Definition: Catalysis of the reaction: 1-O-(4-hydroxy-3-methoxybenzoyl)-beta-D-glucose + cyanidin 3-O-beta-D-glucoside = cyanidin 3,7-di-O-beta-D-glucoside + vanillate. Sources: RHEA:35431